{
  "term_id": "UNKNOWN:0003",
  "gene_symbol": "LRRC9",
  "gene": "UniProtKB:Q6ZRR7",
  "gene_name": "Leucine-rich repeat-containing protein 9",
  "term_label": "Unknown cellular component"
}